{
  "term_id": "UNKNOWN:0001",
  "term_label": "Unknown molecular function",
  "gene": "UniProtKB:A0A0G2JKD1",
  "gene_name": "Mucin-21",
  "gene_symbol": "MUC21"
}